PSII associated light-harvesting complex II, peripheral complex, LHCIIb subcomplex [GO:0030085] (cellular component) Definition: A pigment protein complex that forms part of the photosystem II associated light-harvesting complex II; contains two proteins (usually about 28 and 27 kDa), and may contain a third; peripherally located relative to other LHC polypeptides. References: PMID:8825475 Relationships: is a type of GO:0098807; is part of PSII associated light-harvesting complex II, peripheral complex [GO:0009656]